{
  "gene_symbol": "ZFC3H1",
  "gene": "UniProtKB:O60293",
  "gene_name": "Zinc finger C3H1 domain-containing protein",
  "term_label": "Unknown molecular function",
  "term_id": "UNKNOWN:0001"
}